positive regulation of lateral root development [GO:1901333] (biological process) Sources: GOC:TermGenie Also known as: up regulation of lateral root development, up-regulation of lateral root development, upregulation of lateral root development, activation of lateral root development Relationships: is_a positive regulation of post-embryonic development [GO:0048582]; is a type of regulation of lateral root development [GO:2000023]; positively regulates GO:0048527 Definition: Any process that activates or increases the frequency, rate or extent of lateral root development.